{
  "gene_name": "Microtubule-associated protein 1S",
  "gene": "UniProtKB:Q66K74",
  "term_id": "GO:0043025",
  "gene_symbol": "MAP1S",
  "term_label": "neuronal cell body"
}